pollen coat [GO:0070505] (cellular component) Relationships: is a type of specialized extracellular matrix [GO:0140047] Also known as: pollenkitt, tryphine References: PMID:12930826, PMID:15012271, PMID:28955324 Sources: GOC:mah, GOC:rph Definition: A layer of extracellular matrix deposited onto the surface of the pollen wall upon disintegration of the tapetal layer of the anther wall in the late stages of pollen development. The composition of this material is highly heterogeneous and includes waxes, lipid droplets, small aromatic molecules, and proteins. The pollen coat is proposed to have many functions, such as holding pollen in the anther until dispersal, facilitation of pollen dispersal, protection of pollen from water loss and UV radiation, and facilitation of adhesion of pollen to the stigma.